{
  "gene_symbol": "PAX9",
  "gene_name": "Paired box protein Pax-9",
  "term_id": "GO:0000981",
  "term_label": "DNA-binding transcription factor activity, RNA polymerase II-specific",
  "gene": "UniProtKB:P55771"
}